negative regulation of large conductance calcium-activated potassium channel activity [GO:1902607] (biological process) Definition: Any process that stops, prevents or reduces the frequency, rate or extent of large conductance calcium-activated potassium channel activity. Relationships: is_a negative regulation of potassium ion transmembrane transporter activity [GO:1901017]; negatively regulates large conductance calcium-activated potassium channel activity [GO:0060072] References: PMID:23407708 Sources: GOC:TermGenie, GO_REF:0000059 Also known as: down regulation of BK KCa channels, down regulation of BK calcium-activated potassium channel activity, down regulation of large conductance KCa channels, down regulation of large conductance calcium-activated potassium channel activity, down-regulation of BK KCa channels, down-regulation of BK calcium-activated potassium channel activity, down-regulation of large conductance KCa channels, down-regulation of large conductance calcium-activated potassium channel activity, downregulation of BK KCa channels, downregulation of BK calcium-activated potassium channel activity, downregulation of large conductance KCa channels, downregulation of large conductance calcium-activated potassium channel activity, negative regulation of BK KCa channels, negative regulation of BK calcium-activated potassium channel activity, negative regulation of large conductance KCa channels, inhibition of BK KCa channels, inhibition of BK calcium-activated potassium channel activity, inhibition of large conductance KCa channels, inhibition of large conductance calcium-activated potassium channel activity, down regulation of BK channel activity, down-regulation of BK channel activity, downregulation of BK channel activity, inhibition of BK channel activity, negative regulation of BK channel activity